{
  "gene_name": "Cholesteryl ester transfer protein",
  "gene_symbol": "CETP",
  "term_label": "cholesterol metabolic process",
  "term_id": "GO:0008203",
  "gene": "UniProtKB:P11597"
}